{
  "gene_name": "Zinc finger C3HC-type protein 1",
  "term_label": "nucleus",
  "term_id": "GO:0005634",
  "gene": "UniProtKB:Q86WB0",
  "gene_symbol": "ZC3HC1"
}